{
  "term_id": "GO:0005783",
  "gene_name": "ER lumen protein-retaining receptor 3",
  "gene": "UniProtKB:O43731",
  "term_label": "endoplasmic reticulum",
  "gene_symbol": "KDELR3"
}